angiogenic sprout fusion [GO:0120077] (biological process) References: PMID:28264837 Sources: GOC:cvs Relationships: is a type of anatomical structure formation involved in morphogenesis [GO:0048646]; is part of sprouting angiogenesis [GO:0002040]; has part cell adhesion involved in sprouting angiogenesis [GO:0120078] Definition: The connection of an angiogenic sprout to another vessel or sprout during the formation of vascular networks by sprouting angiogenesis. Also known as: blood vessel anastomosis